TDP catabolic process [GO:0006245] (biological process) Definition: The chemical reactions and pathways resulting in the breakdown of TDP, ribosylthymine diphosphate. Relationships: is a type of GO:0009195; is a type of pyrimidine ribonucleotide catabolic process [GO:0009222]; is a type of TDP metabolic process [GO:0046043] Also known as: TDP breakdown, TDP catabolism, TDP degradation Sources: ISBN:0198506732